{
  "gene_name": "Pleckstrin-2",
  "gene": "UniProtKB:Q9NYT0",
  "term_label": "plasma membrane",
  "term_id": "GO:0005886",
  "gene_symbol": "PLEK2"
}